{
  "gene_name": "Target of EGR1 protein 1",
  "gene_symbol": "TOE1",
  "gene": "UniProtKB:Q96GM8",
  "term_label": "snRNA 3'-end processing",
  "term_id": "GO:0034472"
}